{
  "term_label": "cytoplasm",
  "gene": "UniProtKB:P31152",
  "gene_name": "Mitogen-activated protein kinase 4",
  "term_id": "GO:0005737",
  "gene_symbol": "MAPK4"
}